deoxynucleotide 3'-phosphatase activity [GO:0047846] (molecular function) Definition: Catalysis of the reaction: a deoxynucleoside 3'-phosphate + H2O = a deoxynucleoside + phosphate. Sources: EC:3.1.3.34, MetaCyc:DEOXYNUCLEOTIDE-3-PHOSPHATASE-RXN Relationships: is a type of GO:0016791 Also known as: 3'-deoxynucleotidase activity, 3'-deoxyribonucleotidase activity, deoxyribonucleotide 3'-phosphohydrolase activity